bicyclomycin transmembrane transporter activity [GO:0015545] (molecular function) Relationships: is a type of transmembrane transporter activity [GO:0022857]; is part of bicyclomycin transmembrane transport [GO:0015905] Sources: ISBN:091191028X Also known as: bicyclomycin transporter activity, bicyclomycin/sulfathiazole:hydrogen antiporter activity Definition: Enables the transfer of bicyclomycin from one side of a membrane to the other. Bicyclomycin (or bicozamycin) is an antibacterial drug often used as a livestock feed additive.